{
  "gene_name": "Ubiquitin carboxyl-terminal hydrolase 33",
  "gene": "UniProtKB:Q8TEY7",
  "gene_symbol": "USP33",
  "term_id": "GO:0007399",
  "term_label": "nervous system development"
}